{
  "gene_symbol": "DEFB108C",
  "gene": "UniProtKB:A8MXU0",
  "gene_name": "Putative beta-defensin 108A",
  "term_id": "UNKNOWN:0003",
  "term_label": "Unknown cellular component"
}